{
  "gene": "UniProtKB:A6NDL7",
  "term_label": "protein methyltransferase activity",
  "gene_symbol": "METTL21EP",
  "gene_name": "Putative methyltransferase-like protein 21E pseudogene",
  "term_id": "GO:0008276"
}